{
  "gene_name": "Protein phosphatase 1E",
  "term_id": "GO:0004722",
  "gene": "UniProtKB:Q8WY54",
  "gene_symbol": "PPM1E",
  "term_label": "protein serine/threonine phosphatase activity"
}